{
  "gene_name": "Sorting nexin-20",
  "term_label": "Unknown biological process",
  "gene": "UniProtKB:Q7Z614",
  "term_id": "UNKNOWN:0002",
  "gene_symbol": "SNX20"
}